{
  "gene": "UniProtKB:O00124",
  "term_label": "Unknown cellular component",
  "term_id": "UNKNOWN:0003",
  "gene_symbol": "UBXN8",
  "gene_name": "UBX domain-containing protein 8"
}